MAP kinase phosphatase activity [GO:0033549] (molecular function) Relationships: is a type of phosphoprotein phosphatase activity [GO:0004721] Definition: Catalysis of the reaction: a phosphorylated MAP kinase + H2O = a MAP kinase + phosphate. References: PMID:12184814, PMID:17208316 Sources: GOC:mah Also known as: MAPK phosphatase activity Subtypes: GO:0017017, MAP kinase tyrosine phosphatase activity [GO:0033550], MAP kinase serine/threonine phosphatase activity [GO:1990439]